{
  "term_id": "GO:1990904",
  "gene_name": "RNA-binding protein 12B",
  "gene": "UniProtKB:Q8IXT5",
  "term_label": "ribonucleoprotein complex",
  "gene_symbol": "RBM12B"
}